{
  "gene": "UniProtKB:Q17RF5",
  "term_id": "UNKNOWN:0001",
  "gene_symbol": "ODAPH",
  "term_label": "Unknown molecular function",
  "gene_name": "Odontogenesis associated phosphoprotein"
}